{
  "term_id": "GO:0003333",
  "gene_name": "Putative sodium-coupled neutral amino acid transporter 8",
  "gene": "UniProtKB:A6NNN8",
  "gene_symbol": "SLC38A8",
  "term_label": "amino acid transmembrane transport"
}